{
  "gene": "UniProtKB:Q9H0B6",
  "term_id": "GO:0005737",
  "term_label": "cytoplasm",
  "gene_name": "Kinesin light chain 2",
  "gene_symbol": "KLC2"
}